regulation of atrial cardiac muscle cell membrane repolarization [GO:0060372] (biological process) Also known as: regulation of atrial cardiac muscle cell repolarization, regulation of atrial cardiomyocyte membrane repolarization, atrial repolarization, electrocardiogram QRS complex Sources: GOC:dph, GOC:tb Relationships: is a type of regulation of cardiac muscle cell membrane repolarization [GO:0099623]; regulates atrial cardiac muscle cell membrane repolarization [GO:0099624] Subtypes: regulation of membrane repolarization during atrial cardiac muscle cell action potential [GO:1905000] Definition: Any process that modulates the establishment or extent of a membrane potential in the polarizing direction towards the resting potential in an atrial cardiomyocyte.